interleukin-26 production [GO:0032630] (biological process) Definition: The appearance of interleukin-26 due to biosynthesis or secretion following a cellular stimulus, resulting in an increase in its intracellular or extracellular levels. Relationships: is a type of GO:0001816 Sources: GOC:mah Regulation: regulated by GO:0032670; negatively regulated by negative regulation of interleukin-26 production [GO:0032710]; positively regulated by positive regulation of interleukin-26 production [GO:0032750] Also known as: IL-26 production, AK155 secretion, interleukin-26 anabolism, interleukin-26 biosynthesis, interleukin-26 biosynthetic process, interleukin-26 formation, interleukin-26 secretion, interleukin-26 synthesis